{
  "gene_name": "Zinc finger CCHC domain-containing protein 10",
  "term_id": "UNKNOWN:0002",
  "gene": "UniProtKB:Q8TBK6",
  "term_label": "Unknown biological process",
  "gene_symbol": "ZCCHC10"
}